positive regulation of glucose catabolic process to lactate via pyruvate [GO:1904025] (biological process) Definition: Any process that activates or increases the frequency, rate or extent of glucose catabolic process to lactate via pyruvate. References: PMID:20935145 Sources: GOC:TermGenie, GOC:dph, GO_REF:0000058 Relationships: is a type of GO:0009896; is a type of positive regulation of glucose metabolic process [GO:0010907]; is a type of regulation of glucose catabolic process to lactate via pyruvate [GO:1904023]; positively regulates GO:0019661 Also known as: positive regulation of glucose fermentation to lactate via pyruvate, positive regulation of homofermentation, positive regulation of homofermentative lactate fermentation, positive regulation of homofermentative pathway, positive regulation of homolactate fermentation, positive regulation of homolactic fermentation, up regulation of glucose catabolic process to lactate via pyruvate, up regulation of glucose fermentation to lactate via pyruvate, up regulation of homofermentation, up regulation of homofermentative lactate fermentation, up regulation of homofermentative pathway, up regulation of homolactate fermentation, up regulation of homolactic fermentation, up-regulation of glucose catabolic process to lactate via pyruvate, up-regulation of glucose fermentation to lactate via pyruvate, up-regulation of homofermentation, up-regulation of homofermentative lactate fermentation, up-regulation of homofermentative pathway, up-regulation of homolactate fermentation, up-regulation of homolactic fermentation, upregulation of glucose catabolic process to lactate via pyruvate, upregulation of glucose fermentation to lactate via pyruvate, upregulation of homofermentation, upregulation of homofermentative lactate fermentation, upregulation of homofermentative pathway, upregulation of homolactate fermentation, upregulation of homolactic fermentation, activation of glucose catabolic process to lactate via pyruvate, activation of glucose fermentation to lactate via pyruvate, activation of homofermentation, activation of homofermentative lactate fermentation, activation of homofermentative pathway, activation of homolactate fermentation, activation of homolactic fermentation